{
  "term_id": "GO:0007030",
  "gene_symbol": "TJAP1",
  "term_label": "Golgi organization",
  "gene": "UniProtKB:Q5JTD0",
  "gene_name": "Tight junction-associated protein 1"
}